positive regulation of membrane depolarization during cardiac muscle cell action potential [GO:1900827] (biological process) Definition: Any process that activates or increases the frequency, rate or extent of membrane depolarization during a cardiac muscle cell action potential. Sources: GOC:BHF, GOC:TermGenie, GOC:mtg_cardiac_conduct_nov11 Also known as: up regulation of membrane depolarization during cardiac muscle cell action potential, up-regulation of membrane depolarization during cardiac muscle cell action potential, upregulation of membrane depolarization during cardiac muscle cell action potential, activation of membrane depolarization during cardiac muscle cell action potential Relationships: is a type of regulation of membrane depolarization during cardiac muscle cell action potential [GO:1900825]; is a type of positive regulation of membrane depolarization [GO:1904181]; positively regulates membrane depolarization during cardiac muscle cell action potential [GO:0086012] Subtypes: positive regulation of membrane depolarization during AV node cell action potential [GO:1905029]